{
  "gene_symbol": "NIPA2",
  "gene": "UniProtKB:Q8N8Q9",
  "term_label": "Unknown molecular function",
  "gene_name": "Magnesium transporter NIPA2",
  "term_id": "UNKNOWN:0001"
}